ribonucleoside triphosphate phosphatase activity [GO:0017111] (molecular function) Relationships: is a type of pyrophosphatase activity [GO:0016462] Also known as: apyrase activity, nucleoside 5-triphosphatase activity, nucleoside triphosphatase activity, nucleoside triphosphate hydrolase activity, nucleoside triphosphate phosphatase activity, nucleoside-triphosphatase activity, NTPase activity, nucleoside triphosphate phosphohydrolase activity, nucleoside-5-triphosphate phosphohydrolase activity Sources: RHEA:23680 Regulation: regulated by nucleoside-triphosphatase regulator activity [GO:0060589] Definition: Catalysis of the reaction: a ribonucleoside triphosphate + H2O = a ribonucleoside diphosphate + H+ + phosphate. Subtypes: GTPase activity [GO:0003924], ATP hydrolysis activity [GO:0016887], CTPase activity [GO:0043273], TTPase activity [GO:0050339], ITPase activity [GO:0103023]